lactate aldolase activity [GO:0050041] (molecular function) Definition: Catalysis of the reaction: (S)-lactate = acetaldehyde + formate. Also known as: (S)-lactate acetaldehyde-lyase (formate-forming), (S)-lactate acetaldehyde-lyase activity, lactate synthase activity Relationships: is a type of aldehyde-lyase activity [GO:0016832] Sources: EC:4.1.2.36, RHEA:17909